{
  "gene": "UniProtKB:Q8TE73",
  "term_label": "9+2 motile cilium",
  "term_id": "GO:0097729",
  "gene_name": "Dynein axonemal heavy chain 5",
  "gene_symbol": "DNAH5"
}